{
  "gene_symbol": "PPRC1",
  "term_id": "GO:0097009",
  "term_label": "energy homeostasis",
  "gene": "UniProtKB:Q5VV67",
  "gene_name": "Peroxisome proliferator-activated receptor gamma coactivator-related protein 1"
}